{
  "gene": "UniProtKB:Q11201",
  "gene_symbol": "ST3GAL1",
  "term_id": "GO:0097503",
  "term_label": "sialylation",
  "gene_name": "CMP-N-acetylneuraminate-beta-galactosamide-alpha-2,3-sialyltransferase 1"
}